{
  "gene": "UniProtKB:P61006",
  "term_label": "synaptic vesicle",
  "term_id": "GO:0008021",
  "gene_name": "Ras-related protein Rab-8A",
  "gene_symbol": "RAB8A"
}